{
  "term_label": "Unknown cellular component",
  "gene_name": "IQ domain-containing protein K",
  "gene": "UniProtKB:Q8N0W5",
  "gene_symbol": "IQCK",
  "term_id": "UNKNOWN:0003"
}